{
  "gene": "UniProtKB:P27352",
  "gene_name": "Cobalamin binding intrinsic factor",
  "gene_symbol": "CBLIF",
  "term_label": "cobalamin transport",
  "term_id": "GO:0015889"
}